{
  "term_id": "UNKNOWN:0002",
  "term_label": "Unknown biological process",
  "gene_name": "TBC1 domain family member 2A",
  "gene": "UniProtKB:Q9BYX2",
  "gene_symbol": "TBC1D2"
}